postsynapse [GO:0098794] (cellular component) Sources: GOC:dos Definition: The part of a synapse that is part of the post-synaptic cell. Subtypes: GO:0043197, GO:0098975 Relationships: is_a cellular anatomical structure [GO:0110165]; is part of synapse [GO:0045202]